{
  "gene_symbol": "MAPK3",
  "term_label": "protein serine/threonine kinase activity",
  "gene": "UniProtKB:P27361",
  "gene_name": "Mitogen-activated protein kinase 3",
  "term_id": "GO:0004674"
}